{
  "term_id": "GO:0006002",
  "gene_name": "Glutamine--fructose-6-phosphate aminotransferase [isomerizing] 1",
  "gene_symbol": "GFPT1",
  "gene": "UniProtKB:Q06210",
  "term_label": "fructose 6-phosphate metabolic process"
}